{
  "term_id": "GO:0004510",
  "gene_name": "Tryptophan 5-hydroxylase 1",
  "gene_symbol": "TPH1",
  "term_label": "tryptophan 5-monooxygenase activity",
  "gene": "UniProtKB:P17752"
}